{
  "term_label": "nucleus",
  "term_id": "GO:0005634",
  "gene": "UniProtKB:Q96KK5",
  "gene_name": "Histone H2A type 1-H",
  "gene_symbol": "H2AC12"
}